phosphatidylinositol 5-phosphate metabolic process [GO:1904562] (biological process) References: PMID:23916588 Sources: GOC:PARL, GOC:TermGenie, GOC:autophagy, GOC:dph, GOC:pad Definition: The chemical reactions and pathways involving phosphatidylinositol 5-phosphate. Subtypes: GO:1904563 Relationships: is a type of phosphatidylinositol metabolic process [GO:0046488] Also known as: phosphatidylinositol 5-phosphate metabolism